{
  "gene_name": "Very-long-chain enoyl-CoA reductase",
  "term_label": "sphingolipid metabolic process",
  "gene": "UniProtKB:Q9NZ01",
  "term_id": "GO:0006665",
  "gene_symbol": "TECR"
}